glucosylglycerol metabolic process [GO:0051472] (BP) Subtypes: glucosylglycerol biosynthetic process [GO:0051473] Also known as: glucosylglycerol metabolism Relationships: is a type of GO:0016137; is a type of polyol metabolic process [GO:0019751]; is a type of GO:0044042 Sources: GOC:ai Definition: The chemical reactions and pathways involving glucosylglycerol, alpha-D-glucopyranosyl-alpha-(1,2)-glycerol.